cardiac glial cell differentiation [GO:0060950] (biological process) Definition: The process in which a relatively unspecialized cell acquires the specialized features of a glial cell of the heart. Sources: GOC:mtg_heart Subtypes: GO:0060951 Relationships: is a type of glial cell differentiation [GO:0010001]; is a type of cardiocyte differentiation [GO:0035051]